tyrosine:tyramine antiporter activity [GO:0070908] (molecular function) Also known as: tyrosine-tyramine antiporter activity, tyrosine/tyramine antiporter activity Definition: Catalysis of the reaction: tyrosine(out) + tyramine(in) = tyrosine(in) + tyramine(out). Relationships: is a type of L-tyrosine transmembrane transporter activity [GO:0005302]; is a type of monoamine transmembrane transporter activity [GO:0008504]; is a type of antiporter activity [GO:0015297] Sources: GOC:dh